{
  "term_label": "Unknown molecular function",
  "gene": "UniProtKB:Q96ET8",
  "term_id": "UNKNOWN:0001",
  "gene_symbol": "TVP23C",
  "gene_name": "Golgi apparatus membrane protein TVP23 homolog C"
}